{
  "term_label": "DNA-binding transcription factor activity, RNA polymerase II-specific",
  "gene": "UniProtKB:Q8N3J9",
  "gene_name": "Zinc finger protein 664",
  "term_id": "GO:0000981",
  "gene_symbol": "ZNF664"
}